{
  "term_id": "GO:0005886",
  "gene_symbol": "SLC31A2",
  "gene_name": "Protein SLC31A2",
  "term_label": "plasma membrane",
  "gene": "UniProtKB:O15432"
}